regulation of negative chemotaxis [GO:0050923] (BP) Definition: Any process that modulates the frequency, rate or extent of the directed movement of a motile cell or organism towards a lower concentration in a concentration gradient of a specific chemical. Relationships: is a type of regulation of chemotaxis [GO:0050920]; regulates GO:0050919 Sources: GOC:ai Subtypes: positive regulation of negative chemotaxis [GO:0050924], GO:0050925